cellular bud scar [GO:0005621] (cellular component) Definition: Crater-like ring of chitinous scar tissue located on the surface of the mother cell. It is formed after the newly emerged daughter cell separates thereby marking the site of cytokinesis and septation. The number of bud scars that accumulate on the surface of a cell is a useful determinant of replicative age. Relationships: is a type of GO:0110165; is part of fungal-type cell wall [GO:0009277] References: PMID:14600225, PMID:2005820 Sources: GOC:rn